{
  "term_label": "positive regulation of cell population proliferation",
  "term_id": "GO:0008284",
  "gene_symbol": "FGF18",
  "gene": "UniProtKB:O76093",
  "gene_name": "Fibroblast growth factor 18"
}